regulation of extracellular matrix organization [GO:1903053] (biological process) Also known as: regulation of extracellular matrix organisation, regulation of extracellular matrix organization and biogenesis Definition: Any process that modulates the frequency, rate or extent of extracellular matrix organization. References: PMID:22357537 Sources: GOC:BHF, GOC:TermGenie, GOC:rl, GO_REF:0000058 Subtypes: GO:0003330, GO:0010715, regulation of basement membrane organization [GO:0110011], regulation of extracellular matrix assembly [GO:1901201], negative regulation of extracellular matrix organization [GO:1903054], positive regulation of extracellular matrix organization [GO:1903055], regulation of collagen fibril organization [GO:1904026] Relationships: is a type of GO:0051128; regulates extracellular matrix organization [GO:0030198]